regulation of alpha-glucan biosynthetic process [GO:0032949] (biological process) Relationships: is a type of regulation of glucan biosynthetic process [GO:0010962]; is a type of GO:0032948; regulates alpha-glucan biosynthetic process [GO:0030979] Sources: GOC:mah Also known as: regulation of alpha-glucan anabolism, regulation of alpha-glucan biosynthesis, regulation of alpha-glucan formation, regulation of alpha-glucan synthesis Subtypes: regulation of (1->3)-alpha-glucan biosynthetic process [GO:0070606] Definition: Any process that modulates the frequency, rate or extent of the chemical reactions and pathways relusting in the formation of alpha-glucans.